{
  "term_label": "circadian rhythm",
  "term_id": "GO:0007623",
  "gene_symbol": "RBM4",
  "gene_name": "RNA-binding protein 4",
  "gene": "UniProtKB:Q9BWF3"
}